{
  "term_id": "GO:0005509",
  "term_label": "calcium ion binding",
  "gene": "UniProtKB:P27824",
  "gene_symbol": "CANX",
  "gene_name": "Calnexin"
}